{
  "gene_symbol": "SMAD3",
  "term_id": "GO:0000978",
  "term_label": "RNA polymerase II cis-regulatory region sequence-specific DNA binding",
  "gene": "UniProtKB:P84022",
  "gene_name": "Mothers against decapentaplegic homolog 3"
}